{
  "gene_name": "Interferon alpha-5",
  "term_id": "GO:0002323",
  "gene": "UniProtKB:P01569",
  "gene_symbol": "IFNA5",
  "term_label": "natural killer cell activation involved in immune response"
}